{
  "gene_name": "Centriole, cilia and spindle-associated protein",
  "gene_symbol": "CCSAP",
  "term_id": "GO:0008017",
  "gene": "UniProtKB:Q6IQ19",
  "term_label": "microtubule binding"
}